{
  "term_id": "UNKNOWN:0003",
  "gene_name": "Transmembrane epididymal protein 1",
  "gene": "UniProtKB:Q5T9Z0",
  "term_label": "Unknown cellular component",
  "gene_symbol": "TEDDM1"
}